{
  "gene_name": "Inner nuclear membrane protein Man1",
  "gene_symbol": "LEMD3",
  "term_label": "Unknown biological process",
  "term_id": "UNKNOWN:0002",
  "gene": "UniProtKB:Q9Y2U8"
}